regulation of cyclic nucleotide catabolic process [GO:0030805] (BP) Also known as: regulation of cyclic nucleotide breakdown, regulation of cyclic nucleotide catabolism, regulation of cyclic nucleotide degradation Definition: Any process that modulates the frequency, rate or extent of the chemical reactions and pathways resulting in the breakdown of cyclic nucleotides. Relationships: is a type of GO:0030811; regulates cyclic nucleotide catabolic process [GO:0009214] Sources: GOC:mah